haloacetate dehalogenase activity [GO:0018785] (molecular function) Also known as: haloacetate halidohydrolase activity, monohaloacetate dehalogenase activity Relationships: is a type of hydrolase activity, acting on acid halide bonds, in C-halide compounds [GO:0019120] Definition: Catalysis of the reaction: haloacetate + H2O = glycolate + halide. Sources: EC:3.8.1.3